{
  "gene_symbol": "TFPT",
  "gene_name": "TCF3 fusion partner",
  "term_id": "GO:0003677",
  "gene": "UniProtKB:P0C1Z6",
  "term_label": "DNA binding"
}